{
  "term_id": "GO:0005902",
  "gene_name": "Fascin",
  "gene_symbol": "FSCN1",
  "term_label": "microvillus",
  "gene": "UniProtKB:Q16658"
}